{
  "term_id": "GO:0017056",
  "gene": "UniProtKB:Q96KW2",
  "term_label": "structural constituent of nuclear pore",
  "gene_symbol": "POM121L2",
  "gene_name": "POM121-like protein 2"
}